{
  "gene": "UniProtKB:Q8IW03",
  "gene_symbol": "SIAH3",
  "term_id": "GO:0005737",
  "term_label": "cytoplasm",
  "gene_name": "Seven in absentia homolog 3"
}